{
  "gene": "UniProtKB:Q6UXV1",
  "gene_symbol": "IZUMO2",
  "gene_name": "Izumo sperm-egg fusion protein 2",
  "term_label": "Unknown cellular component",
  "term_id": "UNKNOWN:0003"
}